{
  "gene_symbol": "SPARC",
  "gene_name": "SPARC",
  "term_label": "semicircular canal morphogenesis",
  "term_id": "GO:0048752",
  "gene": "UniProtKB:P09486"
}